{
  "gene": "UniProtKB:Q86XS8",
  "term_id": "GO:0006511",
  "gene_name": "E3 ubiquitin-protein ligase RNF130",
  "term_label": "ubiquitin-dependent protein catabolic process",
  "gene_symbol": "RNF130"
}